protein localization to ciliary transition zone [GO:1904491] (biological process) Definition: A process in which a protein is transported to, or maintained in, a location within a ciliary transition zone. References: PMID:21422230 Sources: GOC:TermGenie, GOC:kmv, GO_REF:0000087 Also known as: protein localisation in ciliary transition zone, protein localisation to ciliary transition zone, protein localization in ciliary transition zone Relationships: is a type of protein localization to cilium [GO:0061512] Subtypes: protein localization to photoreceptor connecting cilium [GO:1903621]